{
  "gene_symbol": "UNC93B1",
  "gene_name": "Protein unc-93 homolog B1",
  "term_id": "GO:0035325",
  "gene": "UniProtKB:Q9H1C4",
  "term_label": "Toll-like receptor binding"
}